{
  "gene_symbol": "FXR2",
  "term_id": "GO:0010494",
  "gene_name": "RNA-binding protein FXR2",
  "gene": "UniProtKB:P51116",
  "term_label": "cytoplasmic stress granule"
}